extracellularly glutamate-gated chloride channel activity [GO:0008068] (molecular function) Also known as: extracellular-glutamate-gated chloride channel activity Definition: Enables the transmembrane transfer of a chloride ion by a channel that opens when glutamate is bound by the channel complex or one of its constituent parts on the extracellular side of the plasma membrane. Relationships: is_a extracellularly glutamate-gated ion channel activity [GO:0005234]; is a type of GO:0005254; is_a GO:0099095 Note: Note that this term represents an activity and not a gene product. Consider also annotating to the molecular function term 'glutamate receptor activity ; GO:0008066'. Sources: GOC:mtg_transport, ISBN:0815340729